{
  "gene_symbol": "SPIRE1",
  "term_id": "GO:0048193",
  "gene_name": "Protein spire homolog 1",
  "gene": "UniProtKB:Q08AE8",
  "term_label": "Golgi vesicle transport"
}